{
  "gene_name": "2-methoxy-6-polyprenyl-1,4-benzoquinol methylase, mitochondrial",
  "term_id": "GO:0006744",
  "gene": "UniProtKB:Q5HYK3",
  "term_label": "ubiquinone biosynthetic process",
  "gene_symbol": "COQ5"
}